CD8-positive, alpha-beta T cell homeostasis [GO:0160165] (BP) Definition: The process of regulating the proliferation and elimination of CD8-positive alpha-beta T cells such that the total number of CD8-positive alpha-beta T cells within a whole or part of an organism is stable over time in the absence of an outside stimulus. References: PMID:30650357, PMID:33815406 Also known as: CD8+ T cell homeostasis, CD8-positive T cell homeostasis Relationships: is a type of T cell homeostasis [GO:0043029]